{
  "gene_symbol": "MTRNR2L6",
  "term_label": "receptor antagonist activity",
  "term_id": "GO:0048019",
  "gene": "UniProtKB:P0CJ73",
  "gene_name": "Humanin-like 6"
}